eupatolide synthase activity [GO:0106244] (molecular function) References: PMID:29758164 Sources: GOC:eab, RHEA:57972 Definition: Catalysis of the reaction: 8beta-hydroxygermacra-1(10),4,11(13)-trien-12-oate + O2 + reduced [NADPH--hemoprotein reductase] = eupatolide + 2 H2O + oxidized [NADPH--hemoprotein reductase]. Relationships: is a type of monooxygenase activity [GO:0004497]